{
  "gene": "UniProtKB:Q9NPF4",
  "gene_name": "tRNA N6-adenosine threonylcarbamoyltransferase",
  "gene_symbol": "OSGEP",
  "term_label": "Unknown molecular function",
  "term_id": "UNKNOWN:0001"
}